{
  "gene_symbol": "GLP1R",
  "gene": "UniProtKB:P43220",
  "term_id": "GO:0017046",
  "gene_name": "Glucagon-like peptide 1 receptor",
  "term_label": "peptide hormone binding"
}